{
  "term_label": "chromosome segregation",
  "gene_name": "Protein phosphatase 1 regulatory subunit 7",
  "term_id": "GO:0007059",
  "gene_symbol": "PPP1R7",
  "gene": "UniProtKB:Q15435"
}